{
  "gene_name": "Serine_arginine-rich splicing factor 11",
  "gene_symbol": "SRSF11",
  "term_id": "GO:0003723",
  "gene": "UniProtKB:Q05519",
  "term_label": "RNA binding"
}